{
  "gene": "UniProtKB:Q03426",
  "gene_name": "Mevalonate kinase",
  "term_label": "mevalonate kinase activity",
  "term_id": "GO:0004496",
  "gene_symbol": "MVK"
}